positive regulation of mRNA alternative polyadenylation [GO:0140409] (biological process) Relationships: is a type of GO:0031442; is a type of regulation of mRNA alternative polyadenylation [GO:0140408]; positively regulates mRNA alternative polyadenylation [GO:0110104] Definition: Any process that activates or increases the frequency, rate or extent of mRNA alternative polyadenylation. References: PMID:29507755